cellular response to reversine [GO:0072764] (biological process) Relationships: is a type of cellular response to purine-containing compound [GO:0071415]; is a type of response to reversine [GO:1901596] Definition: Any process that results in a change in state or activity of a cell (in terms of movement, secretion, enzyme production, gene expression, etc.) as a result of a reversine stimulus. Sources: GOC:mah